{
  "term_id": "GO:0008146",
  "term_label": "sulfotransferase activity",
  "gene_name": "Carbohydrate sulfotransferase 13",
  "gene": "UniProtKB:Q8NET6",
  "gene_symbol": "CHST13"
}